{
  "term_id": "GO:0032970",
  "term_label": "regulation of actin filament-based process",
  "gene_name": "Costars family protein ABRACL",
  "gene_symbol": "ABRACL",
  "gene": "UniProtKB:Q9P1F3"
}